replication fork arrest at tRNA locus [GO:0090001] (biological process) Sources: GOC:dph, GOC:tb Relationships: is a type of replication fork arrest [GO:0043111] Definition: A process that impedes the progress of the DNA replication fork at natural replication fork pausing sites within the eukaryotic tRNA transcription unit.